{
  "gene_symbol": "CD44",
  "term_id": "GO:0016323",
  "gene": "UniProtKB:P16070",
  "gene_name": "CD44 antigen",
  "term_label": "basolateral plasma membrane"
}